{
  "term_label": "protein serine/threonine phosphatase activity",
  "gene": "UniProtKB:Q8NI37",
  "gene_symbol": "PPTC7",
  "gene_name": "Protein phosphatase PTC7 homolog",
  "term_id": "GO:0004722"
}